{
  "gene_symbol": "NBPF11",
  "term_id": "UNKNOWN:0001",
  "gene": "UniProtKB:Q86T75",
  "term_label": "Unknown molecular function",
  "gene_name": "Neuroblastoma breakpoint family member 11"
}